{
  "term_label": "detection of calcium ion",
  "gene": "UniProtKB:Q16558",
  "gene_symbol": "KCNMB1",
  "gene_name": "Calcium-activated potassium channel subunit beta-1",
  "term_id": "GO:0005513"
}